cell differentiation involved in pronephros development [GO:0039014] (biological process) Relationships: is a type of cell differentiation involved in kidney development [GO:0061005]; BFO_0000050 GO:0048793 Sources: GOC:mtg_kidney_jan10 Subtypes: pronephric nephron tubule epithelial cell differentiation [GO:0035778] Definition: The process in which relatively unspecialized cells acquire specialized structural and/or functional features that characterize the cells of the pronephros as it progresses from its formation to the mature state. Also known as: cell differentiation involved in pronephric kidney development